{
  "term_label": "chloride transmembrane transport",
  "term_id": "GO:1902476",
  "gene_symbol": "ANO2",
  "gene_name": "Anoctamin-2",
  "gene": "UniProtKB:Q9NQ90"
}